{
  "gene_name": "Melanoma-associated antigen 3",
  "term_id": "GO:0005634",
  "gene": "UniProtKB:P43357",
  "gene_symbol": "MAGEA3",
  "term_label": "nucleus"
}